{
  "term_label": "phosphatidylinositol-mediated signaling",
  "gene": "UniProtKB:O00443",
  "gene_symbol": "PIK3C2A",
  "term_id": "GO:0048015",
  "gene_name": "Phosphatidylinositol 4-phosphate 3-kinase C2 domain-containing subunit alpha"
}